{
  "term_id": "GO:0045505",
  "term_label": "dynein intermediate chain binding",
  "gene": "UniProtKB:Q8TE73",
  "gene_name": "Dynein axonemal heavy chain 5",
  "gene_symbol": "DNAH5"
}